{
  "gene_name": "Ral GTPase-activating protein subunit alpha-1",
  "gene": "UniProtKB:Q6GYQ0",
  "term_label": "cytoplasm",
  "term_id": "GO:0005737",
  "gene_symbol": "RALGAPA1"
}